{
  "gene_symbol": "SLC14A1",
  "gene": "UniProtKB:Q13336",
  "gene_name": "Urea transporter 1",
  "term_id": "UNKNOWN:0003",
  "term_label": "Unknown cellular component"
}